{
  "gene_symbol": "OR52H1",
  "term_id": "UNKNOWN:0002",
  "gene": "UniProtKB:Q8NGJ2",
  "gene_name": "Olfactory receptor 52H1",
  "term_label": "Unknown biological process"
}